medium-chain fatty acid-CoA ligase activity [GO:0031956] (molecular function) Definition: Catalysis of the reaction: a medium-chain fatty acid + ATP + CoA = a medium-chain fatty acyl-CoA + AMP + diphosphate. A medium-chain fatty acid has an aliphatic tail containing 6 to 12 carbons. Also known as: medium-chain fatty-acid-CoA ligase activity, medium-chain-fatty-acid-CoA ligase activity, medium-chain fatty acid activation Relationships: is a type of fatty acid-CoA ligase activity [GO:0120515] Sources: RHEA:48340 Note: While there is not universal consensus on the lengths of short-, medium-, long- and very-long-chain fatty acids, the GO uses the definitions in ChEBI (see CHEBI:26666, CHEBI:59554, CHEBI:15904 and CHEBI:27283). Subtypes: decanoate-CoA ligase activity [GO:0102391]